{
  "gene_name": "Tyrosine-protein kinase Mer",
  "term_label": "receptor complex",
  "gene_symbol": "MERTK",
  "term_id": "GO:0043235",
  "gene": "UniProtKB:Q12866"
}